{
  "term_id": "GO:0005783",
  "gene": "UniProtKB:Q9BT40",
  "term_label": "endoplasmic reticulum",
  "gene_name": "Inositol polyphosphate 5-phosphatase K",
  "gene_symbol": "INPP5K"
}